{
  "gene_symbol": "TMEM156",
  "gene_name": "Transmembrane protein 156",
  "term_label": "Unknown molecular function",
  "term_id": "UNKNOWN:0001",
  "gene": "UniProtKB:Q8N614"
}